{
  "term_label": "Unknown biological process",
  "term_id": "UNKNOWN:0002",
  "gene_name": "Axonemal dynein light chain domain-containing protein 1",
  "gene": "UniProtKB:Q5T1B0",
  "gene_symbol": "AXDND1"
}